{
  "term_label": "canonical Wnt signaling pathway",
  "gene_symbol": "FZD4",
  "gene_name": "Frizzled-4",
  "term_id": "GO:0060070",
  "gene": "UniProtKB:Q9ULV1"
}